{
  "gene_name": "Coiled-coil domain-containing protein 66",
  "gene_symbol": "CCDC66",
  "gene": "UniProtKB:A2RUB6",
  "term_id": "GO:0005929",
  "term_label": "cilium"
}